auditory behavior [GO:0031223] (biological process) Also known as: auditory behaviour, behavioral response to sound, behavioural response to sound Sources: GOC:pr, GOC:rc Subtypes: vocal learning [GO:0042297] Relationships: is a type of GO:0007638; BFO_0000050 GO:0010996 Definition: The behavior of an organism in response to a sound.